{
  "gene_symbol": "WASH2P",
  "gene": "UniProtKB:Q6VEQ5",
  "term_label": "WASH complex",
  "term_id": "GO:0071203",
  "gene_name": "WAS protein family homolog 2"
}